(+)-sabinol dehydrogenase activity [GO:0047502] (MF) Sources: EC:1.1.1.228, RHEA:18329 Definition: Catalysis of the reaction: (+)-cis-sabinol + NAD+ = (1S,5S)-sabinone + H+ + NADH. Also known as: (+)-cis-sabinol dehydrogenase activity, (+)-cis-sabinol:NAD+ oxidoreductase activity Relationships: is a type of oxidoreductase activity, acting on the CH-OH group of donors, NAD or NADP as acceptor [GO:0016616]